{
  "term_label": "phosphatidylinositol transfer activity",
  "term_id": "GO:0008526",
  "gene_name": "Membrane-associated phosphatidylinositol transfer protein 1",
  "gene_symbol": "PITPNM1",
  "gene": "UniProtKB:O00562"
}